{
  "term_id": "UNKNOWN:0001",
  "gene_name": "Distal membrane-arm assembly complex protein 1",
  "gene_symbol": "DMAC1",
  "gene": "UniProtKB:Q96GE9",
  "term_label": "Unknown molecular function"
}